{
  "gene": "UniProtKB:P35858",
  "gene_symbol": "IGFALS",
  "gene_name": "Insulin-like growth factor-binding protein complex acid labile subunit",
  "term_id": "GO:0038023",
  "term_label": "signaling receptor activity"
}